{
  "gene": "UniProtKB:P29371",
  "term_label": "plasma membrane",
  "gene_symbol": "TACR3",
  "term_id": "GO:0005886",
  "gene_name": "Neuromedin-K receptor"
}